kievitone hydratase activity [GO:0050015] (molecular function) Sources: EC:4.2.1.95, RHEA:23604 Definition: Catalysis of the reaction: kievitone hydrate = H2O + H+ + kievitone. Also known as: KHase activity, kievitone-hydrate hydro-lyase (kievitone-forming), kievitone-hydrate hydro-lyase activity Relationships: is a type of hydro-lyase activity [GO:0016836]